{
  "gene_symbol": "PON1",
  "gene_name": "Serum paraoxonase_arylesterase 1",
  "term_id": "GO:0004063",
  "term_label": "aryldialkylphosphatase activity",
  "gene": "UniProtKB:P27169"
}